negative regulation of transporter activity [GO:0032410] (biological process) Also known as: down regulation of transporter activity, down-regulation of transporter activity, downregulation of transporter activity, inhibition of transporter activity Subtypes: negative regulation of ion transmembrane transporter activity [GO:0032413] Relationships: is a type of negative regulation of molecular function [GO:0044092]; is_a negative regulation of transport [GO:0051051]; negatively regulates transporter activity [GO:0005215] Definition: Any process that stops or reduces the activity of a transporter. Sources: GOC:mah